{
  "term_id": "GO:0017158",
  "gene_symbol": "SYT15B",
  "gene": "UniProtKB:X6R8R1",
  "gene_name": "Synaptotagmin-15B",
  "term_label": "regulation of calcium ion-dependent exocytosis"
}